regulation of erythrocyte apoptotic process [GO:1902250] (biological process) Definition: Any process that modulates the frequency, rate or extent of erythrocyte apoptotic process. References: PMID:14569084 Sources: GOC:BHF, GOC:TermGenie, GOC:mtg_apoptosis, GOC:rl Also known as: regulation of RBC apoptotic process, regulation of red blood cell apoptotic process, regulation of RBC apoptosis, regulation of erythrocyte apoptosis, regulation of red blood cell apoptosis Relationships: is_a regulation of myeloid cell apoptotic process [GO:0033032]; regulates erythrocyte apoptotic process [GO:1902217] Subtypes: negative regulation of erythrocyte apoptotic process [GO:1902251], GO:1902252